{
  "term_id": "GO:0090575",
  "term_label": "RNA polymerase II transcription regulator complex",
  "gene": "UniProtKB:O00716",
  "gene_name": "Transcription factor E2F3",
  "gene_symbol": "E2F3"
}